pheromone activity [GO:0005186] (molecular function) Definition: The activity of binding to and activating specific cell surface receptors, thereby inducing behavioral, developmental, or physiological response(s) from a responding organism or cell. The substance may be released or retained on the cell surface. Pheromones may serve as a specific attractant, social communicator, or sexual stimulant. Subtypes: mating pheromone activity [GO:0000772], competence pheromone activity [GO:0030413] Sources: GOC:sgd_curators, ISBN:0198506732 Relationships: is a type of GO:0048018; BFO_0000051 signaling receptor binding [GO:0005102] Note: Also consider annotating to 'receptor agonist activity ; GO:0048018'.